sepal giant cell differentiation [GO:0090392] (biological process) References: PMID:20485493 Sources: GOC:tb Relationships: is a type of plant epidermal cell differentiation [GO:0090627] Definition: The process in which a relatively unspecialized cell acquires specialized features of a sepal giant cell. A sepal giant cell is a pavement cell that is part of the sepal epidermis and stretches one fifth the length of the sepal with a chromosome content of 16C.